mitotic sister chromatid cohesion [GO:0007064] (biological process) Relationships: is a type of sister chromatid cohesion [GO:0007062] Definition: The cell cycle process in which the sister chromatids of a replicated chromosome are joined along the entire length of the chromosome, from their formation in S phase through metaphase during a mitotic cell cycle. This cohesion cycle is critical for high fidelity chromosome transmission. References: PMID:10827941, PMID:11389843, PMID:14623866 Sources: GOC:ai, GOC:rn Subtypes: GO:0071961, mitotic sister chromatid cohesion, centromeric [GO:0071962], mitotic sister chromatid cohesion, telomeric [GO:0099404]